{
  "gene": "UniProtKB:B1AKI9",
  "term_label": "Unknown molecular function",
  "gene_name": "Isthmin-1",
  "gene_symbol": "ISM1",
  "term_id": "UNKNOWN:0001"
}